oxidoreductase activity, reducing C-O-C group as acceptor [GO:0120546] (molecular function) Subtypes: GO:0010283, GO:0010284, violaxanthin de-epoxidase activity [GO:0046422] Sources: EC:1.23.-.- Relationships: is a type of oxidoreductase activity [GO:0016491] Definition: Catalysis of an oxidation-reduction (redox) reaction in which a reducing C-O-C group acts as acceptor.